{
  "gene_name": "Collagen alpha-2(VIII) chain",
  "gene": "UniProtKB:P25067",
  "term_label": "extracellular matrix organization",
  "term_id": "GO:0030198",
  "gene_symbol": "COL8A2"
}